{
  "gene_name": "Protein boule-like",
  "gene_symbol": "BOLL",
  "term_id": "GO:0045948",
  "gene": "UniProtKB:Q8N9W6",
  "term_label": "positive regulation of translational initiation"
}